RNA guanylyltransferase activity [GO:0008192] (molecular function) Relationships: is a type of guanylyltransferase activity [GO:0070568]; is a type of catalytic activity, acting on RNA [GO:0140098] Sources: GOC:mah Definition: Catalysis of the posttranscriptional addition of a guanyl residue to the 5' end of an RNA molecule. Subtypes: mRNA guanylyltransferase activity [GO:0004484], GO:0008193